{
  "gene": "UniProtKB:Q8IZ81",
  "term_id": "UNKNOWN:0003",
  "gene_name": "ELMO domain-containing protein 2",
  "gene_symbol": "ELMOD2",
  "term_label": "Unknown cellular component"
}